eisosome [GO:0032126] (cellular component) Definition: A cell part that is composed of the eisosome membrane or MCC domain, a furrow-like plasma membrane sub-domain and associated integral transmembrane proteins, and the proteins (eisosome filaments) that form a scaffolding lattice on the cytoplasmic face. Eisosomes broadly affect overall plasma membrane organization. References: PMID:16496001, PMID:22368779 Sources: GOC:al, GOC:vw Relationships: is_a cellular anatomical structure [GO:0110165]